{
  "term_label": "Unknown biological process",
  "gene": "UniProtKB:Q9Y6N7",
  "gene_symbol": "ROBO1",
  "gene_name": "Roundabout homolog 1",
  "term_id": "UNKNOWN:0002"
}